choline O-acetyltransferase activity [GO:0004102] (molecular function) Also known as: CHOACTase activity, acetyl-CoA:choline O-acetyltransferase activity, choline acetylase activity, choline acetyltransferase activity Relationships: is a type of O-acetyltransferase activity [GO:0016413] Sources: EC:2.3.1.6, RHEA:18821 Definition: Catalysis of the reaction: acetyl-CoA + choline = acetylcholine + CoA.